ribonuclease T1 activity [GO:0046589] (molecular function) Definition: Catalysis of the endonucleolytic cleavage to nucleoside 3'-phosphates and 3'-phosphooligonucleotides ending in Gp with 2',3'-cyclic phosphate intermediates. Also known as: RNase T1 activity, ribonuclease F1, Aspergillus oryzae ribonuclease activity, RNase F1, RNase G, RNase N1 activity, RNase N2 activity, RNase Sa, RNase T1, binase activity, guanyl-specific RNase activity, guanyloribonuclease activity, ribonuclease C2, ribonuclease Ch, ribonuclease N1, ribonuclease N3, ribonuclease PP1, ribonuclease SA, ribonuclease U1, ribonuclease guaninenucleotido-2'-transferase (cyclizing) Relationships: is a type of RNA endonuclease activity [GO:0004521]; is_a phosphorus-oxygen lyase activity [GO:0016849] Sources: EC:4.6.1.24